{
  "gene_name": "Ras-related GTP-binding protein C",
  "gene": "UniProtKB:Q9HB90",
  "gene_symbol": "RRAGC",
  "term_id": "GO:0005764",
  "term_label": "lysosome"
}